{
  "term_id": "GO:0035567",
  "gene_symbol": "SFRP5",
  "term_label": "non-canonical Wnt signaling pathway",
  "gene_name": "Secreted frizzled-related protein 5",
  "gene": "UniProtKB:Q5T4F7"
}